regulation of purine nucleotide catabolic process [GO:0033121] (biological process) Also known as: regulation of purine nucleotide breakdown, regulation of purine nucleotide catabolism, regulation of purine nucleotide degradation Definition: Any process that modulates the frequency, rate or extent of the chemical reactions and pathways resulting in the breakdown of purine nucleotides. Subtypes: regulation of glycolytic process [GO:0006110], negative regulation of purine nucleotide catabolic process [GO:0033122], positive regulation of purine nucleotide catabolic process [GO:0033123] Relationships: is a type of regulation of nucleotide catabolic process [GO:0030811]; is a type of regulation of purine nucleotide metabolic process [GO:1900542]; RO_0002211 purine nucleotide catabolic process [GO:0006195] Sources: GOC:mah